{
  "gene_name": "Transmembrane protein 185B",
  "term_id": "UNKNOWN:0003",
  "gene": "UniProtKB:Q9H7F4",
  "term_label": "Unknown cellular component",
  "gene_symbol": "TMEM185B"
}